{
  "gene_name": "Protein phosphatase 1 regulatory subunit 12C",
  "term_label": "cytoplasm",
  "gene": "UniProtKB:Q9BZL4",
  "term_id": "GO:0005737",
  "gene_symbol": "PPP1R12C"
}